{
  "term_label": "membrane",
  "term_id": "GO:0016020",
  "gene_symbol": "NBEAL1",
  "gene": "UniProtKB:Q6ZS30",
  "gene_name": "Neurobeachin-like protein 1"
}